synaptic vesicle, resting pool [GO:1990476] (cellular component) Also known as: reserve pool of synaptic vesicles, resting pool of synaptic vesicles Definition: A synaptic vesicle belonging to the pool that remain unreleased even after prolonged stimulation causes a saturating degree of vesicular turnover. 50-80% of the total number of synaptic vesicles at a resting terminal bouton are in this pool. Relationships: is a type of synaptic vesicle [GO:0008021]; is part of terminal bouton [GO:0043195] References: PMID:22745285 Sources: GOC:pad